positive regulation of blood coagulation, intrinsic pathway [GO:2000268] (BP) Relationships: is a type of positive regulation of blood coagulation [GO:0030194]; is a type of positive regulation of protein activation cascade [GO:2000259]; is a type of GO:2000266; positively regulates blood coagulation, intrinsic pathway [GO:0007597] Definition: Any process that activates or increases the frequency, rate or extent of blood coagulation, intrinsic pathway. Sources: GOC:mah